protein branching point deglutamylation [GO:0035611] (biological process) References: PMID:21074048 Sources: GOC:sp Relationships: is a type of protein deglutamylation [GO:0035608] Definition: The removal of a branching point glutamate residue. A branching point glutamate connects a glutamate side chain to a gene-encoded glutamate residue.